{
  "gene_symbol": "SEC24B",
  "gene_name": "Protein transport protein Sec24B",
  "term_id": "GO:0000149",
  "gene": "UniProtKB:O95487",
  "term_label": "SNARE binding"
}